{
  "term_label": "cis-Golgi network",
  "gene_name": "Golgin subfamily A member 8S",
  "gene_symbol": "GOLGA8S",
  "term_id": "GO:0005801",
  "gene": "UniProtKB:H3BPF8"
}